{
  "gene": "UniProtKB:Q16828",
  "term_id": "GO:0070373",
  "term_label": "negative regulation of ERK1 and ERK2 cascade",
  "gene_symbol": "DUSP6",
  "gene_name": "Dual specificity protein phosphatase 6"
}